antibody-dependent cellular cytotoxicity [GO:0001788] (biological process) Also known as: ADCC, antibody dependent cell death, antibody dependent cell killing, antibody-dependent cell death, antibody-dependent cell killing, type VI hypersensitivity Regulation: regulated by GO:0001813; negatively regulated by negative regulation of antibody-dependent cellular cytotoxicity [GO:0001814]; RO_0002213 by positive regulation of antibody-dependent cellular cytotoxicity [GO:0001815] Relationships: is a type of GO:0001794; is a type of leukocyte mediated cytotoxicity [GO:0001909] References: PMID:11677095, PMID:9581795 Sources: GOC:pr, ISBN:0781735149 Definition: Cytolysis of target cells by natural killer cells, eosinophils, neutrophils, monocytes, or macrophages following engagement of antibodies bound to the target cells by Fc receptors on the effector cells.